positive regulation of pyroptotic inflammatory response [GO:0140639] (biological process) Definition: Any process that increases the frequency, rate or extent of a pyroptotic inflammatory response. References: PMID:24626226 Also known as: positive regulation of pyroptosis Relationships: is_a positive regulation of inflammatory response [GO:0050729]; positively regulates pyroptotic inflammatory response [GO:0070269]